heme oxygenase (decyclizing) activity [GO:0004392] (molecular function) Definition: Catalysis of the reaction: heme b + 3 O2 + 3 reduced [NADPH-hemoprotein reductase] = biliverdin + CO + Fe2+ + H+ + 3 H2O + 3 oxidized [NADPH-hemoprotein reductase]. Sources: RHEA:21764 Also known as: haem oxygenase (decyclizing) activity, ORP33 proteins, haem oxidase activity, haem oxygenase activity, heme oxidase activity, heme oxygenase activity, heme,hydrogen-donor:oxygen oxidoreductase (alpha-methene-oxidizing, hydroxylating) Relationships: is a type of oxidoreductase activity, acting on paired donors, with incorporation or reduction of molecular oxygen, reduced flavin or flavoprotein as one donor, and incorporation of one atom of oxygen [GO:0016712]